{
  "gene": "UniProtKB:P0DMT0",
  "term_label": "Unknown molecular function",
  "gene_symbol": "MRLN",
  "term_id": "UNKNOWN:0001",
  "gene_name": "Myoregulin"
}